{
  "gene": "UniProtKB:Q96RQ3",
  "gene_name": "Methylcrotonoyl-CoA carboxylase subunit alpha, mitochondrial",
  "term_id": "GO:0004485",
  "term_label": "methylcrotonoyl-CoA carboxylase activity",
  "gene_symbol": "MCCC1"
}